{
  "term_label": "GTPase activity",
  "gene_name": "Immunity-related GTPase family M protein",
  "gene": "UniProtKB:A1A4Y4",
  "term_id": "GO:0003924",
  "gene_symbol": "IRGM"
}